short-chain fatty acid-CoA ligase activity [GO:0031955] (molecular function) Definition: Catalysis of the reaction: a short-chain fatty acid + ATP + CoA = a short-chain fatty acyl-CoA + AMP + diphosphate. A short-chain fatty acid has an aliphatic tail containing fewer than 6 carbons. References: PMID:34904027 Sources: RHEA:52860 Also known as: short-chain fatty-acid-CoA ligase activity, short-chain-fatty-acid-CoA ligase activity, short-chain fatty acid activation Relationships: is a type of fatty acid-CoA ligase activity [GO:0120515] Note: While there is not universal consensus on the lengths of short-, medium-, long- and very-long-chain fatty acids, the GO uses the definitions in ChEBI (see CHEBI:26666, CHEBI:59554, CHEBI:15904 and CHEBI:27283). Subtypes: 2-methylbutanoate-CoA ligase activity [GO:0043759], propionate-CoA ligase activity [GO:0050218]